{
  "gene": "UniProtKB:Q96B42",
  "term_label": "Unknown biological process",
  "term_id": "UNKNOWN:0002",
  "gene_name": "Transmembrane protein 18",
  "gene_symbol": "TMEM18"
}